{
  "term_label": "positive regulation of cell population proliferation",
  "gene_name": "Epigen",
  "gene_symbol": "EPGN",
  "term_id": "GO:0008284",
  "gene": "UniProtKB:Q6UW88"
}